{
  "term_id": "UNKNOWN:0001",
  "gene": "UniProtKB:Q7Z7B0",
  "gene_name": "Filamin-A-interacting protein 1",
  "gene_symbol": "FILIP1",
  "term_label": "Unknown molecular function"
}